tRNA-5-taurinomethyluridine 2-sulfurtransferase [GO:0061708] (molecular function) Relationships: is a type of sulfurtransferase activity [GO:0016783]; is a type of catalytic activity, acting on a tRNA [GO:0140101] References: PMID:15509579 Sources: GOC:dph, RHEA:47040 Definition: Catalysis of 5-taurinomethyluridine in tRNA + a [protein]-S-sulfanylcysteine + ATP + a reduced electron acceptor = a 5-taurinomethyl-2-thiouridine in tRNA + a [protein]-L-cysteine + AMP + an oxidized electron acceptor + diphosphate + H+.